S-adenosyl-L-methionine:(S)-corytuberine-N-methyltransferase activity [GO:0102964] (molecular function) Relationships: is a type of methyltransferase activity [GO:0008168] Definition: Catalysis of the reaction: (S)-corytuberine + S-adenosyl-L-methionine = magnoflorine + S-adenosyl-L-homocysteine. Sources: RHEA:51524